{
  "term_id": "GO:0007411",
  "gene_symbol": "EMB",
  "gene_name": "Embigin",
  "gene": "UniProtKB:Q6PCB8",
  "term_label": "axon guidance"
}